{
  "gene_name": "Neutral amino acid uniporter 4",
  "gene_symbol": "SLC36A4",
  "gene": "UniProtKB:Q6YBV0",
  "term_label": "amino acid transmembrane transport",
  "term_id": "GO:0003333"
}